{
  "term_label": "Unknown molecular function",
  "gene_name": "Shieldin complex subunit 1",
  "gene_symbol": "SHLD1",
  "gene": "UniProtKB:Q8IYI0",
  "term_id": "UNKNOWN:0001"
}